{
  "gene": "UniProtKB:Q96R28",
  "term_id": "GO:0004984",
  "term_label": "olfactory receptor activity",
  "gene_symbol": "OR2M2",
  "gene_name": "Olfactory receptor 2M2"
}